{
  "term_id": "UNKNOWN:0001",
  "gene_symbol": "PLEKHM3",
  "gene": "UniProtKB:Q6ZWE6",
  "gene_name": "Pleckstrin homology domain-containing family M member 3",
  "term_label": "Unknown molecular function"
}